glycine:sodium symporter activity [GO:0015375] (molecular function) Relationships: is a type of neutral L-amino acid:sodium symporter activity [GO:0005295]; is a type of organic acid:sodium symporter activity [GO:0005343]; is a type of GO:0015187 Sources: GOC:ai Definition: Enables the transfer of a solute or solutes from one side of a membrane to the other according to the reaction: glycine(out) + Na+(out) = glycine(in) + Na+(in).